{
  "gene_symbol": "HYI",
  "term_label": "Unknown cellular component",
  "gene": "UniProtKB:Q5T013",
  "gene_name": "Putative hydroxypyruvate isomerase",
  "term_id": "UNKNOWN:0003"
}